etioplast membrane [GO:0034426] (cellular component) Definition: Either of the lipid bilayers that surround a etioplast and form the etioplast envelope. Sources: GOC:rph Relationships: is a type of plastid membrane [GO:0042170]; is part of etioplast envelope [GO:0034425]